oxygen evolving activity [GO:0010242] (molecular function) Also known as: photosynthetic water oxidation Relationships: is a type of oxidoreductase activity [GO:0016491] Definition: Catalysis of the reaction: 2 H2O = O2 + 4 H+ + 4 e-. The evolution of oxygen from oxidizing water is carried out by the oxygen evolving complex in photosystem II of plants. P680+, the photochemically oxidized reaction-center chlorophyll of PSII, is a strong biological oxidant. The reduction potential of P680+ is more positive than that of water, and thus it can oxidize water to give O2 and H+ ions. The oxygen escapes as a gas while the H+ ions remain in solution inside the thylakoid vesicle. References: PMID:17091926, PMID:7948862 Sources: GOC:kd, GOC:syr